{
  "gene_symbol": "BARHL1",
  "gene": "UniProtKB:Q9BZE3",
  "term_label": "RNA polymerase II transcription regulatory region sequence-specific DNA binding",
  "gene_name": "BarH-like 1 homeobox protein",
  "term_id": "GO:0000977"
}